{
  "gene_symbol": "BOD1L2",
  "gene": "UniProtKB:Q8IYS8",
  "gene_name": "Biorientation of chromosomes in cell division protein 1-like 2",
  "term_label": "Unknown biological process",
  "term_id": "UNKNOWN:0002"
}